{
  "term_id": "GO:0005513",
  "term_label": "detection of calcium ion",
  "gene_name": "Calcium-activated potassium channel subunit beta-2",
  "gene_symbol": "KCNMB2",
  "gene": "UniProtKB:Q9Y691"
}